{
  "gene_symbol": "AGBL1",
  "gene_name": "Cytosolic carboxypeptidase 4",
  "term_label": "metallocarboxypeptidase activity",
  "term_id": "GO:0004181",
  "gene": "UniProtKB:Q96MI9"
}